clathrin-sculpted glutamate transport vesicle [GO:0060199] (cellular component) Relationships: is a type of transport vesicle [GO:0030133]; is a type of clathrin-sculpted vesicle [GO:0060198] Sources: GOC:dph Definition: A clathrin-sculpted lipid bilayer membrane-enclosed vesicle after clathrin release and containing glutamate. Also known as: clathrin sculpted glutamate constitutive secretory pathway transport vesicle, clathrin sculpted glutamate transport vesicle